putrescine acetylation [GO:0032920] (biological process) Relationships: is a type of putrescine metabolic process [GO:0009445]; is a type of polyamine acetylation [GO:0032917] Sources: GOC:mlg Definition: The modification of putrescine by addition of acetyl groups.